regulation of extrathymic T cell differentiation [GO:0033082] (biological process) Definition: Any process that modulates the frequency, rate or extent of extrathymic T cell differentiation. Also known as: regulation of extrathymic T cell development Relationships: is a type of regulation of T cell differentiation [GO:0045580]; RO_0002211 extrathymic T cell differentiation [GO:0033078] Subtypes: GO:0033086, positive regulation of extrathymic T cell differentiation [GO:0033090] Note: Note that immunologists typically use the word 'development' to refer to cells of B or T cell lineages undergoing the process that GO describes as 'cell differentiation'. Sources: GOC:add, GOC:mah